{
  "term_id": "GO:0006396",
  "gene_symbol": "ADARB1",
  "gene_name": "Double-stranded RNA-specific editase 1",
  "term_label": "RNA processing",
  "gene": "UniProtKB:P78563"
}